{
  "term_id": "GO:0072344",
  "gene_symbol": "ZNF598",
  "gene": "UniProtKB:Q86UK7",
  "term_label": "rescue of stalled ribosome",
  "gene_name": "E3 ubiquitin-protein ligase ZNF598"
}